{
  "gene_symbol": "CD84",
  "gene": "UniProtKB:Q9UIB8",
  "gene_name": "SLAM family member 5",
  "term_id": "UNKNOWN:0001",
  "term_label": "Unknown molecular function"
}